TTPase activity [GO:0050339] (molecular function) Relationships: is a type of ribonucleoside triphosphate phosphatase activity [GO:0017111] Sources: RHEA:19013 Also known as: thymidine triphosphatase activity, thymidine-triphosphatase activity, dTTP nucleotidohydrolase activity, dTTPase activity, deoxythymidine-5'-triphosphatase activity, thymidine triphosphate nucleotidohydrolase activity Definition: Catalysis of the reaction: dTTP + H2O = dTDP + H+ + phosphate.